{
  "term_id": "GO:0048821",
  "gene_symbol": "HBB",
  "gene_name": "Hemoglobin subunit beta",
  "term_label": "erythrocyte development",
  "gene": "UniProtKB:P68871"
}